protein transmembrane transport [GO:0071806] (biological process) Relationships: is a type of GO:0015031; is a type of transmembrane transport [GO:0055085] Sources: GOC:mah, GOC:vw Also known as: protein membrane transport Definition: The process in which a protein is transported across a membrane. Subtypes: protein import into mitochondrial matrix [GO:0030150], protein secretion by the type I secretion system [GO:0030253], GO:0030254, protein secretion by the type IV secretion system [GO:0030255], protein secretion by the type VI secretion system [GO:0033103], protein transport by the Sec complex [GO:0043952], protein transport by the Tat complex [GO:0043953], protein secretion by the type VII secretion system [GO:0044315], protein import into chloroplast stroma [GO:0045037], protein import into mitochondrial intermembrane space [GO:0045041], GO:0065002, protein transport across the cell outer membrane [GO:0098776], GO:0160303 Note: Note that this term is not intended for use in annotating lateral movement within membranes.